{
  "gene": "UniProtKB:P11142",
  "term_id": "GO:0005829",
  "term_label": "cytosol",
  "gene_symbol": "HSPA8",
  "gene_name": "Heat shock cognate 71 kDa protein"
}